{
  "term_id": "GO:0005789",
  "gene_symbol": "DGAT2",
  "gene": "UniProtKB:Q96PD7",
  "gene_name": "Diacylglycerol O-acyltransferase 2",
  "term_label": "endoplasmic reticulum membrane"
}